{
  "gene_symbol": "B3GNT7",
  "gene": "UniProtKB:Q8NFL0",
  "gene_name": "UDP-GlcNAc:betaGal beta-1,3-N-acetylglucosaminyltransferase 7",
  "term_label": "UDP-glycosyltransferase activity",
  "term_id": "GO:0008194"
}